{
  "gene_name": "RNA-binding protein 39",
  "term_label": "U1 snRNP binding",
  "gene_symbol": "RBM39",
  "gene": "UniProtKB:Q14498",
  "term_id": "GO:1990446"
}